cellular hyperosmotic salinity response [GO:0071475] (biological process) Sources: GOC:mah Relationships: is_a hyperosmotic salinity response [GO:0042538]; is a type of cellular response to salt stress [GO:0071472]; is a type of cellular hyperosmotic response [GO:0071474] Regulation: regulated by regulation of cellular hyperosmotic salinity response [GO:1900069]; negatively regulated by negative regulation of cellular hyperosmotic salinity response [GO:1900070] Also known as: cellular response to hyperosmotic salt stress Definition: Any process that results in a change in state or activity of a cell (in terms of movement, secretion, enzyme production, gene expression, etc.) as a result of detection of, or exposure to, an increase in the concentration of salt (particularly but not exclusively sodium and chloride ions) in the environment.